{
  "gene_symbol": "ADGRG3",
  "gene_name": "Adhesion G protein-coupled receptor G3",
  "gene": "UniProtKB:Q86Y34",
  "term_label": "G protein-coupled receptor signaling pathway",
  "term_id": "GO:0007186"
}